{
  "gene_name": "Double homeobox protein 4",
  "gene": "UniProtKB:Q9UBX2",
  "term_label": "RNA polymerase II transcription regulatory region sequence-specific DNA binding",
  "term_id": "GO:0000977",
  "gene_symbol": "DUX4"
}